L-phenylalaine oxidase activity [GO:0106329] (molecular function) Relationships: is a type of L-amino-acid oxidase activity [GO:0001716] Definition: Catalysis of the reaction: H2O + L-phenylalanine + O2 = 3-phenylpyruvate + H2O2 + NH4(+). Sources: RHEA:61240